{
  "term_label": "nuclear-transcribed mRNA catabolic process",
  "term_id": "GO:0000956",
  "gene_name": "Negative regulator of P-body association",
  "gene": "UniProtKB:A0A0U1RRE5",
  "gene_symbol": "NBDY"
}